{
  "term_label": "acetylcholine receptor signaling pathway",
  "term_id": "GO:0095500",
  "gene": "UniProtKB:P43681",
  "gene_symbol": "CHRNA4",
  "gene_name": "Neuronal acetylcholine receptor subunit alpha-4"
}